{
  "term_id": "UNKNOWN:0001",
  "gene_symbol": "UBE2V1",
  "gene_name": "Ubiquitin-conjugating enzyme E2 variant 1",
  "gene": "UniProtKB:Q13404",
  "term_label": "Unknown molecular function"
}